{
  "term_id": "UNKNOWN:0003",
  "gene_symbol": "UBALD1",
  "gene": "UniProtKB:Q8TB05",
  "gene_name": "UBA-like domain-containing protein 1",
  "term_label": "Unknown cellular component"
}